{
  "gene_name": "ATPase WRNIP1",
  "term_id": "GO:0008047",
  "gene": "UniProtKB:Q96S55",
  "term_label": "enzyme activator activity",
  "gene_symbol": "WRNIP1"
}